cell-cell signaling involved in mesonephros development [GO:0061210] (biological process) Also known as: cell-cell signalling involved in mesonephros development Relationships: is a type of cell-cell signaling involved in kidney development [GO:0060995]; is part of GO:0001823 Definition: Any process that mediates the transfer of information from one cell to another and contributes to the progression of the mesonephros over time, from its formation to the mature organ. Sources: GOC:mtg_kidney_jan10